{
  "gene_symbol": "LAGE3",
  "term_label": "Unknown molecular function",
  "gene_name": "EKC_KEOPS complex subunit LAGE3",
  "term_id": "UNKNOWN:0001",
  "gene": "UniProtKB:Q14657"
}